multicellular organismal locomotion [GO:0071965] (biological process) Sources: GOC:mah Definition: Locomotion in a multicellular organism, i.e. self-propelled movement of a multicellular organism from one location to another. Relationships: is a type of locomotion [GO:0040011]; is a type of GO:0050879